{
  "gene_symbol": "VCPIP1",
  "gene_name": "Deubiquitinating protein VCPIP1",
  "term_id": "UNKNOWN:0003",
  "term_label": "Unknown cellular component",
  "gene": "UniProtKB:Q96JH7"
}